{
  "term_label": "phosphoribosylaminoimidazolecarboxamide formyltransferase activity",
  "gene_symbol": "ATIC",
  "term_id": "GO:0004643",
  "gene": "UniProtKB:P31939",
  "gene_name": "Bifunctional purine biosynthesis protein ATIC"
}